{
  "gene": "UniProtKB:Q8NGX6",
  "term_label": "odorant binding",
  "gene_name": "Olfactory receptor 10R2",
  "term_id": "GO:0005549",
  "gene_symbol": "OR10R2"
}